{
  "gene_symbol": "FPR3",
  "gene": "UniProtKB:P25089",
  "term_id": "GO:0004982",
  "gene_name": "N-formyl peptide receptor 3",
  "term_label": "N-formyl peptide receptor activity"
}